{
  "gene": "UniProtKB:P85298",
  "gene_symbol": "ARHGAP8",
  "gene_name": "Rho GTPase-activating protein 8",
  "term_label": "negative regulation of endocytic recycling",
  "term_id": "GO:2001136"
}